{
  "gene_name": "Homeobox protein Hox-D12",
  "gene": "UniProtKB:P35452",
  "gene_symbol": "HOXD12",
  "term_id": "GO:1990837",
  "term_label": "sequence-specific double-stranded DNA binding"
}